{
  "term_label": "protein tag activity",
  "gene": "UniProtKB:G2XKQ0",
  "gene_name": "Small ubiquitin-related modifier 5",
  "term_id": "GO:0031386",
  "gene_symbol": "SUMO1P1"
}